anterior head segmentation [GO:0035288] (biological process) Also known as: procephalic segmentation Note: See also the fly_anatomy.ontology term 'procephalic segment ; FBbt:00000007' and its children. Relationships: is a type of GO:0035287; is part of anterior head development [GO:0097065] Definition: Partitioning the insect head anlage into procephalic (labral, (ocular), antennal and intercalary) segments. The procephalic segments lie anterior to the gnathal (posterior head) segments, and are pattered by different segmentation gene cascades to the abdominal, thoracic and posterior head (gnathal) segments. References: PMID:15382136